{
  "gene": "UniProtKB:Q6ZMJ2",
  "term_label": "endocytosis",
  "gene_name": "Scavenger receptor class A member 5",
  "gene_symbol": "SCARA5",
  "term_id": "GO:0006897"
}